beta-L-arabinofuranosidase activity [GO:0102478] (molecular function) Sources: GOC:pz, RHEA:36051 Definition: Catalysis of the reaction: beta-L-arabinofuranosyl-(1->2)-beta-L-arabinofuranose + H2O = 2 beta-L-arabinofuranose. Relationships: is a type of hydrolase activity, hydrolyzing O-glycosyl compounds [GO:0004553]